{
  "gene_name": "Transcriptional regulator Kaiso",
  "gene_symbol": "ZBTB33",
  "gene": "UniProtKB:Q86T24",
  "term_id": "GO:0002682",
  "term_label": "regulation of immune system process"
}